{
  "term_id": "GO:0005884",
  "gene_symbol": "CORO1A",
  "term_label": "actin filament",
  "gene_name": "Coronin-1A",
  "gene": "UniProtKB:P31146"
}